{
  "gene_symbol": "PDCL2",
  "gene": "UniProtKB:Q8N4E4",
  "term_id": "UNKNOWN:0001",
  "gene_name": "Phosducin-like protein 2",
  "term_label": "Unknown molecular function"
}